glutamine-tRNA ligase activity [GO:0004819] (molecular function) Definition: Catalysis of the reaction: ATP + L-glutamine + tRNA(Gln) = AMP + diphosphate + L-glutaminyl-tRNA(Gln). Relationships: is a type of aminoacyl-tRNA ligase activity [GO:0004812] Sources: EC:6.1.1.18 Also known as: glutaminyl-tRNA synthetase activity, GlnRS, L-glutamine:tRNAGln ligase (AMP-forming), glutamine translase activity, glutamine-tRNA synthetase activity, glutaminyl ribonucleic acid, glutaminyl-transfer RNA synthetase activity, glutaminyl-transfer ribonucleate synthetase activity